protein-DNA complex remodeling [GO:0001120] (biological process) Definition: The acquisition, loss, or modification of macromolecules within a protein-DNA complex, resulting in the alteration of an existing complex. Subtypes: DNA-templated transcription open complex formation [GO:0001112] Also known as: protein-DNA complex remodelling Relationships: is a type of GO:0034367; is a type of GO:0071824 Sources: GOC:txnOH